{
  "gene": "UniProtKB:Q96CV9",
  "term_id": "GO:0043122",
  "gene_name": "Optineurin",
  "gene_symbol": "OPTN",
  "term_label": "regulation of canonical NF-kappaB signal transduction"
}